{
  "gene": "UniProtKB:Q9UPG8",
  "term_id": "GO:0000981",
  "term_label": "DNA-binding transcription factor activity, RNA polymerase II-specific",
  "gene_name": "Zinc finger protein PLAGL2",
  "gene_symbol": "PLAGL2"
}